leucosome [GO:0043699] (cellular component) Definition: A tissue-specific, membrane-bounded cytoplasmic organelle within which uric acid and/or purines crystalize in reflective stacks. Leucosomes are synthesized in leucophore cells and have a whitish cast. Relationships: is a type of pigment granule [GO:0048770] Also known as: refractosome Sources: GOC:mh